{
  "gene_name": "Soluble calcium-activated nucleotidase 1",
  "gene_symbol": "CANT1",
  "gene": "UniProtKB:Q8WVQ1",
  "term_id": "GO:0030166",
  "term_label": "proteoglycan biosynthetic process"
}